protein localization to presynaptic membrane [GO:0099644] (biological process) Sources: GOC:dos Definition: A process in which a protein is transported to, or maintained in, a location within a presynaptic membrane. Also known as: protein localisation in presynaptic membrane, protein localisation to presynaptic membrane, protein localization in presynaptic membrane Relationships: is a type of protein localization to membrane [GO:0072657]; is a type of GO:1905383; is a type of protein localization to cell periphery [GO:1990778]